{
  "term_id": "GO:0007160",
  "gene": "UniProtKB:P16144",
  "gene_name": "Integrin beta-4",
  "gene_symbol": "ITGB4",
  "term_label": "cell-matrix adhesion"
}